{
  "gene_symbol": "ODC1",
  "term_id": "GO:0005737",
  "gene": "UniProtKB:P11926",
  "term_label": "cytoplasm",
  "gene_name": "Ornithine decarboxylase"
}